protein targeting to vacuole [GO:0006623] (biological process) Relationships: is a type of GO:0006605; is_a intracellular protein transport [GO:0006886]; is a type of vacuolar transport [GO:0007034]; is_a GO:0072665; is a type of establishment of protein localization to vacuole [GO:0072666] Sources: GOC:curators Subtypes: GO:0006622, GO:0032258, protein targeting to vacuolar membrane [GO:0044395], GO:0071211, cytoplasm to vacuole targeting by the NVT pathway [GO:0120113] Definition: The process of directing proteins towards the vacuole, usually using signals contained within the protein. Also known as: protein vacuolar targeting, protein-vacuolar targeting, protein-vacuole targeting, vacuolar protein sorting